{
  "gene_symbol": "STRA8",
  "gene_name": "Stimulated by retinoic acid gene 8 protein homolog",
  "gene": "UniProtKB:Q7Z7C7",
  "term_id": "GO:0005634",
  "term_label": "nucleus"
}